{
  "term_label": "olfactory receptor activity",
  "gene": "UniProtKB:Q8NGZ0",
  "gene_name": "Olfactory receptor 2AJ1",
  "gene_symbol": "OR2AJ1",
  "term_id": "GO:0004984"
}